{
  "gene_symbol": "PTPRJ",
  "term_label": "axon guidance",
  "gene_name": "Receptor-type tyrosine-protein phosphatase eta",
  "term_id": "GO:0007411",
  "gene": "UniProtKB:Q12913"
}